{
  "term_id": "GO:0005737",
  "gene_name": "Beta-arrestin-1",
  "gene_symbol": "ARRB1",
  "term_label": "cytoplasm",
  "gene": "UniProtKB:P49407"
}